{
  "gene_name": "Coagulation factor VII",
  "term_id": "GO:0007596",
  "term_label": "blood coagulation",
  "gene": "UniProtKB:P08709",
  "gene_symbol": "F7"
}